{
  "gene_name": "Spectrin beta chain, non-erythrocytic 1",
  "gene": "UniProtKB:Q01082",
  "term_id": "GO:0030054",
  "term_label": "cell junction",
  "gene_symbol": "SPTBN1"
}